{
  "gene_name": "Protein FAM174C",
  "term_label": "extracellular region",
  "term_id": "GO:0005576",
  "gene": "UniProtKB:Q9BVV8",
  "gene_symbol": "FAM174C"
}